'de novo' pyridoxal 5'-phosphate biosynthetic process [GO:0036001] (biological process) Also known as: 'de novo' pyridoxal phosphate biosynthetic process, 'de novo' PLP biosynthesis, 'de novo' pyridoxal 5'-phosphate anabolism, 'de novo' pyridoxal 5'-phosphate biosynthesis, 'de novo' pyridoxal 5'-phosphate formation, 'de novo' pyridoxal 5'-phosphate synthesis Definition: The chemical reactions and pathways resulting in the formation of pyridoxal 5'-phosphate, the active form of vitamin B6, from simpler components. Sources: GOC:bf, GOC:yaf, MetaCyc:PYRIDOXSYN-PWY Relationships: is a type of pyridoxal phosphate biosynthetic process [GO:0042823]